G protein-coupled receptor dimeric complex [GO:0038037] (CC) References: PMID:10713101 Sources: GOC:al, GOC:bf Also known as: G-protein coupled receptor dimer, G-protein coupled receptor dimeric complex, GPCR dimer Definition: A protein complex that contains two G protein-coupled receptors. Relationships: is a type of GO:0097648 Subtypes: GO:0038038, G protein-coupled receptor heterodimeric complex [GO:0038039], G protein-coupled GABA receptor complex [GO:1902712], adrenomedullin receptor complex [GO:1903143]